7-methylguanosine cap hypermethylation [GO:0036261] (BP) References: PMID:11983179, PMID:18775984 Sources: GOC:BHF, GOC:bf, GOC:krc, GOC:mah, GOC:rl Relationships: is a type of RNA methylation [GO:0001510]; is a type of RNA capping [GO:0036260] Definition: Hypermethylation of the 7-(mono)methylguanosine (m(7)G) cap structure at the 2' position of the guanosine residue to convert a mono-methylated cap to a 2,2,7-trimethylguanosine cap structure. This type of cap modification occurs on small nuclear RNAs (snRNAs) and small nucleolar RNAs (snoRNAs) and is dependent on prior guanine-N7 methylation. Also known as: 2,2,7-trimethylguanosine cap formation, TMG cap formation, conversion of m(7)G to m(3)G, m(7)G cap hypermethylation, hypermethylation of snRNA cap, hypermethylation of snoRNA cap, snRNA capping, snoRNA capping